positive regulation of B cell receptor signaling pathway [GO:0050861] (biological process) Definition: Any process that activates or increases the frequency, rate or extent of signaling pathways initiated by the cross-linking of an antigen receptor on a B cell. Also known as: positive regulation of B cell receptor signalling pathway, positive regulation of B lymphocyte receptor signaling pathway, positive regulation of B lymphocyte receptor signalling pathway, positive regulation of B-cell receptor signaling pathway, positive regulation of B-cell receptor signalling pathway, positive regulation of B-lymphocyte receptor signaling pathway, positive regulation of B-lymphocyte receptor signalling pathway, up regulation of B cell receptor signaling pathway, up-regulation of B cell receptor signaling pathway, upregulation of B cell receptor signaling pathway, activation of B cell receptor signaling pathway, stimulation of B cell receptor signaling pathway Sources: GOC:ai Relationships: is_a regulation of B cell receptor signaling pathway [GO:0050855]; is a type of positive regulation of antigen receptor-mediated signaling pathway [GO:0050857]; positively regulates B cell receptor signaling pathway [GO:0050853]